{
  "gene_name": "Membrane-spanning 4-domains subfamily A member 18",
  "gene": "UniProtKB:Q3C1V0",
  "term_id": "GO:0005886",
  "term_label": "plasma membrane",
  "gene_symbol": "MS4A18"
}